{
  "gene_symbol": "EXOC2",
  "term_label": "Unknown molecular function",
  "gene": "UniProtKB:Q96KP1",
  "term_id": "UNKNOWN:0001",
  "gene_name": "Exocyst complex component 2"
}